{
  "gene_name": "Multifunctional procollagen lysine hydroxylase and glycosyltransferase LH3",
  "gene": "UniProtKB:O60568",
  "gene_symbol": "PLOD3",
  "term_id": "GO:0033823",
  "term_label": "procollagen glucosyltransferase activity"
}